{
  "term_id": "GO:0000932",
  "gene": "UniProtKB:Q96IF1",
  "term_label": "P-body",
  "gene_symbol": "AJUBA",
  "gene_name": "LIM domain-containing protein ajuba"
}